{
  "gene_symbol": "VAMP2",
  "term_id": "GO:0031201",
  "term_label": "SNARE complex",
  "gene_name": "Vesicle-associated membrane protein 2",
  "gene": "UniProtKB:P63027"
}